intracellular membrane-bounded organelle [GO:0043231] (cellular component) Also known as: intracellular membrane-enclosed organelle Subtypes: nucleus [GO:0005634], mitochondrion [GO:0005739], GO:0005773, endoplasmic reticulum [GO:0005783], endoplasmic reticulum-Golgi intermediate compartment [GO:0005793], Golgi apparatus [GO:0005794], cis-Golgi network [GO:0005801], plastid [GO:0009536], ER body [GO:0010168], mitochondrial derivative [GO:0016007], microneme [GO:0020009], acidocalcisome [GO:0020022], GO:0031094, mitosome [GO:0032047], nucleomorph [GO:0033009], attachment organelle [GO:0033099], hydrogenosome [GO:0042566], GO:0042579, endosperm protein body [GO:0042735], anammoxosome [GO:0044222], pirellulosome [GO:0044223], GO:0044227, exoneme [GO:0044311], karyomere [GO:0061468], GO:0070074, GO:0070088, subsynaptic reticulum [GO:0071212], ocelloid [GO:0097693], intracellular vesicle [GO:0097708], magnetosome [GO:0110143], migrasome [GO:0140494], TMEM240-body [GO:0160045], polaroplast [GO:0160201], fibrous body-membranous organelle [GO:0160208], GO:1990413, omegasome [GO:1990462] Relationships: is a type of GO:0043227; is a type of intracellular organelle [GO:0043229] Definition: Organized structure of distinctive morphology and function, bounded by a single or double lipid bilayer membrane and occurring within the cell. Includes the nucleus, mitochondria, plastids, vacuoles, and vesicles. Excludes the plasma membrane. Sources: GOC:go_curators